{
  "term_id": "GO:0004984",
  "gene": "UniProtKB:Q8NGI7",
  "term_label": "olfactory receptor activity",
  "gene_symbol": "OR10V1",
  "gene_name": "Olfactory receptor 10V1"
}